{
  "gene_symbol": "BBS12",
  "term_label": "Unknown molecular function",
  "term_id": "UNKNOWN:0001",
  "gene_name": "Bardet-Biedl syndrome 12 protein",
  "gene": "UniProtKB:Q6ZW61"
}